regulation of testosterone biosynthetic process [GO:2000224] (biological process) Sources: GOC:obol, GOC:yaf Definition: Any process that modulates the frequency, rate or extent of testosterone biosynthetic process. Relationships: is a type of regulation of ketone biosynthetic process [GO:0010566]; is_a regulation of steroid biosynthetic process [GO:0050810]; regulates testosterone biosynthetic process [GO:0061370] Subtypes: negative regulation of testosterone biosynthetic process [GO:2000225]